{
  "gene": "UniProtKB:Q9BVI4",
  "gene_name": "Nucleolar complex protein 4 homolog",
  "term_label": "Noc4p-Nop14p complex",
  "term_id": "GO:0030692",
  "gene_symbol": "NOC4L"
}